{
  "gene": "UniProtKB:Q6P587",
  "gene_name": "Acylpyruvase FAHD1, mitochondrial",
  "term_label": "mitochondrion",
  "term_id": "GO:0005739",
  "gene_symbol": "FAHD1"
}